{
  "gene_symbol": "PTDSS1",
  "term_label": "Unknown cellular component",
  "gene_name": "Phosphatidylserine synthase 1",
  "gene": "UniProtKB:P48651",
  "term_id": "UNKNOWN:0003"
}